regulation of cell cycle process [GO:0010564] (biological process) Definition: Any process that modulates a cellular process that is involved in the progression of biochemical and morphological phases and events that occur in a cell during successive cell replication or nuclear replication events. Subtypes: GO:0007063, regulation of mitotic nuclear division [GO:0007088], regulation of reciprocal meiotic recombination [GO:0010520], regulation of mitotic spindle pole body separation [GO:0010695], GO:0010946, GO:0010948, regulation of centriole-centriole cohesion [GO:0030997], regulation of telomere maintenance via semi-conservative replication [GO:0032213], regulation of cytokinesis [GO:0032465], regulation of DNA endoreduplication [GO:0032875], regulation of spindle elongation [GO:0032887], regulation of cytokinetic process [GO:0032954], regulation of nuclear cell cycle DNA replication [GO:0033262], GO:0034307, regulation of meiotic nuclear division [GO:0040020], regulation of mitotic centrosome separation [GO:0046602], regulation of centrosome cycle [GO:0046605], GO:0051983, GO:0051988, Wnt signaling pathway, regulating spindle positioning [GO:0060069], regulation of ascospore wall beta-glucan biosynthetic process [GO:0060622], regulation of G0 to G1 transition [GO:0070316], GO:0090068, GO:0090173, regulation of spindle organization [GO:0090224], regulation of cell cycle switching, mitotic to meiotic cell cycle [GO:0110044], regulation of chromosome attachment to the nuclear envelope [GO:0120264], regulation of oocyte karyosome formation [GO:0120313], GO:1901987, regulation of ascospore-type prospore membrane formation [GO:1903023], regulation of mitotic recombination-dependent replication fork processing [GO:1903221], regulation of meiotic DNA double-strand break formation [GO:1903341], regulation of mitotic chromosome condensation [GO:1903379], regulation of G1 to G0 transition [GO:1903450], regulation of meiotic cell cycle process involved in oocyte maturation [GO:1903538], regulation of centriole elongation [GO:1903722], GO:1904726, regulation of mitotic nuclear envelope disassembly [GO:1905557] Relationships: is a type of regulation of cell cycle [GO:0051726]; regulates cell cycle process [GO:0022402] Sources: GOC:dph, GOC:tb